{
  "gene": "UniProtKB:P00519",
  "gene_name": "Tyrosine-protein kinase ABL1",
  "term_id": "GO:0007229",
  "gene_symbol": "ABL1",
  "term_label": "integrin-mediated signaling pathway"
}